{
  "gene": "UniProtKB:P46952",
  "term_id": "GO:0005737",
  "term_label": "cytoplasm",
  "gene_symbol": "HAAO",
  "gene_name": "3-hydroxyanthranilate 3,4-dioxygenase"
}